{
  "gene_name": "Histone H2B type 1-M",
  "term_label": "nucleosome",
  "term_id": "GO:0000786",
  "gene": "UniProtKB:Q99879",
  "gene_symbol": "H2BC14"
}